cyclomaltodextrinase activity [GO:0047798] (molecular function) Definition: Catalysis of the reaction: H2O + cyclomaltodextrin = linear maltodextrin. Sources: EC:3.2.1.54, MetaCyc:CYCLOMALTODEXTRINASE-RXN Also known as: cyclodextrinase activity, cycloheptaglucanase activity, cyclohexaglucanase activity, cyclomaltodextrin dextrin-hydrolase (decyclizing) Relationships: is a type of hydrolase activity, hydrolyzing O-glycosyl compounds [GO:0004553]